11-deoxycorticosterone reductase activity [GO:0102635] (molecular function) Sources: GOC:pz, HEA:47716 Definition: Catalysis of the reaction: 11-deoxycorticosterone + NADH + H+ = 4-pregnen-20,21-diol-3-one + NAD. Relationships: is a type of oxidoreductase activity, acting on the CH-OH group of donors, NAD or NADP as acceptor [GO:0016616]